{
  "gene": "UniProtKB:Q8WUW1",
  "gene_name": "Protein BRICK1",
  "term_id": "GO:0048870",
  "term_label": "cell motility",
  "gene_symbol": "BRK1"
}